{
  "gene_symbol": "XIRP1",
  "gene_name": "Xin actin-binding repeat-containing protein 1",
  "term_id": "GO:0005925",
  "gene": "UniProtKB:Q702N8",
  "term_label": "focal adhesion"
}